negative regulation of telomere maintenance via telomere lengthening [GO:1904357] (biological process) Subtypes: GO:0032211 Relationships: is a type of GO:0032205; is a type of GO:1904356; RO_0002212 telomere maintenance via telomere lengthening [GO:0010833] Definition: Any process that stops, prevents or reduces the frequency, rate or extent of telomere maintenance via telomere lengthening. References: PMID:23959892 Sources: GOC:BHF, GOC:BHF_telomere, GOC:TermGenie, GOC:nc, GO_REF:0000058 Also known as: down regulation of telomere maintenance via telomere lengthening, down-regulation of telomere maintenance via telomere lengthening, downregulation of telomere maintenance via telomere lengthening, inhibition of telomere maintenance via telomere lengthening